L-cysteine transaminase activity [GO:0047801] (molecular function) Sources: RHEA:17441 Definition: Catalysis of the reaction: L-cysteine + 2-oxoglutarate = mercaptopyruvate + L-glutamate. Also known as: cysteine aminotransferase activity, L-cysteine:2-oxoglutarate aminotransferase activity, cysteine transaminase activity Relationships: is a type of GO:0008483